{
  "gene": "UniProtKB:P13501",
  "gene_name": "C-C motif chemokine 5",
  "gene_symbol": "CCL5",
  "term_id": "GO:0030335",
  "term_label": "positive regulation of cell migration"
}